regulation of photosynthesis, light reaction [GO:0042548] (biological process) Sources: GOC:jl Definition: Any process that modulates the frequency, rate or extent of the light-dependent reaction of photosynthesis. Relationships: is a type of regulation of photosynthesis [GO:0010109]; is a type of regulation of generation of precursor metabolites and energy [GO:0043467]; regulates photosynthesis, light reaction [GO:0019684] Subtypes: photosystem II stabilization [GO:0042549], GO:0042550, negative regulation of photosynthesis, light reaction [GO:0043155], photosynthetic state transition [GO:0062055]